{
  "term_id": "GO:0030141",
  "gene": "UniProtKB:Q92932",
  "term_label": "secretory granule",
  "gene_symbol": "PTPRN2",
  "gene_name": "Receptor-type tyrosine-protein phosphatase N2"
}